{
  "term_label": "ubiquitin-like ligase-substrate adaptor activity",
  "term_id": "GO:1990756",
  "gene_symbol": "KEAP1",
  "gene": "UniProtKB:Q14145",
  "gene_name": "Kelch-like ECH-associated protein 1"
}